N-carbamoylputrescine amidase activity [GO:0050126] (molecular function) Definition: Catalysis of the reaction: N-carbamoylputrescine + H2O + 2 H+ = CO2 + NH4 + putrescine. Relationships: is a type of hydrolase activity, acting on carbon-nitrogen (but not peptide) bonds, in linear amides [GO:0016811] Sources: EC:3.5.1.53, RHEA:22284 Also known as: N-carbamoylputrescine amidohydrolase activity, NCP, carbamoylputrescine hydrolase activity